{
  "gene": "UniProtKB:Q9BT81",
  "term_label": "nucleus",
  "term_id": "GO:0005634",
  "gene_symbol": "SOX7",
  "gene_name": "Transcription factor SOX-7"
}